{
  "term_id": "GO:0051015",
  "gene": "UniProtKB:P37802",
  "gene_symbol": "TAGLN2",
  "term_label": "actin filament binding",
  "gene_name": "Transgelin-2"
}